regulation of granuloma formation [GO:0002631] (BP) Relationships: is a type of GO:0002676; is a type of regulation of immune effector process [GO:0002697]; regulates GO:0002432 Definition: Any process that modulates the frequency, rate, or extent of granuloma formation. Subtypes: GO:0002632, positive regulation of granuloma formation [GO:0002633] Sources: GOC:add